{
  "term_id": "GO:0031490",
  "gene_name": "Lysine-specific demethylase 3A",
  "term_label": "chromatin DNA binding",
  "gene_symbol": "KDM3A",
  "gene": "UniProtKB:Q9Y4C1"
}